{
  "gene_symbol": "PSPC1",
  "term_id": "GO:0005634",
  "term_label": "nucleus",
  "gene": "UniProtKB:Q8WXF1",
  "gene_name": "Paraspeckle component 1"
}